{
  "gene": "UniProtKB:P20160",
  "gene_symbol": "AZU1",
  "term_label": "extracellular space",
  "term_id": "GO:0005615",
  "gene_name": "Azurocidin"
}